{
  "gene_symbol": "KRTAP9-8",
  "term_id": "UNKNOWN:0002",
  "term_label": "Unknown biological process",
  "gene_name": "Keratin-associated protein 9-8",
  "gene": "UniProtKB:Q9BYQ0"
}